{
  "term_label": "Golgi apparatus",
  "term_id": "GO:0005794",
  "gene_symbol": "CLCN4",
  "gene": "UniProtKB:P51793",
  "gene_name": "H(+)_Cl(-) exchange transporter 4"
}